d-4,5 unsaturated beta-glucuronyl hydrolase activity [GO:0052788] (molecular function) References: PMID:12729728 Sources: GOC:mengo_curators Also known as: unsaturated beta-glucuronyl hydrolase activity Relationships: is a type of hydrolase activity, hydrolyzing O-glycosyl compounds [GO:0004553] Definition: Catalysis of the hydrolysis of the glycosidic bond in an unsaturated saccharide between the unsaturated glucuronyl residue at the nonreducing terminus and the saccharide linked to the residue.